{
  "term_id": "GO:0042554",
  "gene": "UniProtKB:Q9HBY0",
  "gene_name": "NADPH oxidase 3",
  "gene_symbol": "NOX3",
  "term_label": "superoxide anion generation"
}